{
  "gene_name": "Supervillin",
  "term_label": "phosphatidylinositol-4,5-bisphosphate binding",
  "gene_symbol": "SVIL",
  "gene": "UniProtKB:O95425",
  "term_id": "GO:0005546"
}